{
  "gene_symbol": "COPZ2",
  "term_label": "COPI vesicle coat",
  "gene_name": "Coatomer subunit zeta-2",
  "term_id": "GO:0030126",
  "gene": "UniProtKB:Q9P299"
}